myoblast differentiation involved in skeletal muscle regeneration [GO:0014835] (biological process) References: PMID:16607119 Sources: CL:0000056, GOC:ef, GOC:mtg_muscle Relationships: is a type of GO:0045445; is part of skeletal muscle tissue regeneration [GO:0043403] Definition: The process in which a relatively unspecialized satellite cell acquires specialized features of a myoblast. This occurs as part of skeletal muscle regeneration. A myoblast is a mononucleate cell type that, by fusion with other myoblasts, gives rise to the myotubes that eventually develop into skeletal muscle fibers.